fraxetin biosynthesis [GO:0106147] (biological process) References: PMID:29581584 Sources: GOC:lr Relationships: is a type of coumarin biosynthetic process [GO:0009805] Definition: The chemical reactions and pathways resulting in the formation of fraxetin.